xylanosome [GO:1990358] (cellular component) Definition: A multifunctional supermolecular complex, containing several proteins with hemicellulase activity. Functions to hydrolyze hemicellulose. References: PMID:16769147 Sources: GOC:mengo_curators Also known as: xylanolytic complex Relationships: is_a GO:1902494